regulation of glycogen metabolic process [GO:0070873] (biological process) Definition: Any process that modulates the frequency, rate or extent of the chemical reactions and pathways involving glycogen. Sources: GOC:mah Subtypes: GO:0005979, regulation of glycogen catabolic process [GO:0005981], GO:0070874, positive regulation of glycogen metabolic process [GO:0070875] Relationships: is a type of regulation of polysaccharide metabolic process [GO:0032881]; is a type of regulation of generation of precursor metabolites and energy [GO:0043467]; regulates glycogen metabolic process [GO:0005977] Also known as: regulation of glycogen metabolism